{
  "term_label": "regulation of dendritic spine morphogenesis",
  "gene_name": "Rho GTPase-activating protein 32",
  "term_id": "GO:0061001",
  "gene_symbol": "ARHGAP32",
  "gene": "UniProtKB:A7KAX9"
}